{
  "gene_symbol": "H3-3B",
  "term_label": "nucleosome",
  "term_id": "GO:0000786",
  "gene_name": "Histone H3.3",
  "gene": "UniProtKB:P84243"
}